D-methionine-pyruvate transaminase activity [GO:0047306] (MF) Definition: Catalysis of the reaction: D-methionine + pyruvate = 4-methylthio-2-oxobutanoate + L-alanine. Sources: EC:2.6.1.41, RHEA:23836 Also known as: D-methionine-pyruvate aminotransferase activity, D-methionine aminotransferase activity, D-methionine transaminase activity, D-methionine--pyruvate aminotransferase activity, D-methionine:pyruvate aminotransferase activity Relationships: is a type of GO:0008483